{
  "term_id": "GO:0005737",
  "gene": "UniProtKB:Q9NS87",
  "gene_name": "Kinesin-like protein KIF15",
  "gene_symbol": "KIF15",
  "term_label": "cytoplasm"
}